{
  "term_id": "GO:0006805",
  "gene_symbol": "CYP2U1",
  "gene": "UniProtKB:Q7Z449",
  "gene_name": "Cytochrome P450 2U1",
  "term_label": "xenobiotic metabolic process"
}